{
  "term_label": "protein ubiquitination",
  "gene_symbol": "TRAIP",
  "gene_name": "E3 ubiquitin-protein ligase TRAIP",
  "term_id": "GO:0016567",
  "gene": "UniProtKB:Q9BWF2"
}